{
  "gene_symbol": "PCCB",
  "term_id": "GO:0004658",
  "gene_name": "Propionyl-CoA carboxylase beta chain, mitochondrial",
  "gene": "UniProtKB:P05166",
  "term_label": "propionyl-CoA carboxylase activity"
}